dihydropterin oxidase activity [GO:0004154] (molecular function) Definition: Catalysis of the reaction: a 7,8-dihydropteridine compound + O2 = an oxidized 7,8-dihydropteridine compound + H2O2. Specific substrates and their fully oxidized products include: 7,8-dihydropteridin/pterin, 7,8-dihydrobiopterin/biopterin, 7,8-dihydroxanthopterin/xanthopterin and sepiapterin/oxidized sepiapterin. References: PMID:1745247, PMID:38786926, PMID:6815189 Sources: GOC:sjm Relationships: is a type of oxidoreductase activity, acting on the CH-NH group of donors, oxygen as acceptor [GO:0016647]